{
  "gene_symbol": "RNF151",
  "term_id": "UNKNOWN:0003",
  "gene": "UniProtKB:Q2KHN1",
  "gene_name": "RING finger protein 151",
  "term_label": "Unknown cellular component"
}